{
  "gene_symbol": "PLK5",
  "term_label": "kinetochore",
  "term_id": "GO:0000776",
  "gene_name": "Inactive serine_threonine-protein kinase PLK5",
  "gene": "UniProtKB:Q496M5"
}